{
  "term_label": "IRE1-TRAF2-ASK1 complex",
  "gene_symbol": "TRAF2",
  "term_id": "GO:1990604",
  "gene_name": "TNF receptor-associated factor 2",
  "gene": "UniProtKB:Q12933"
}